{
  "term_label": "negative regulation of DNA-templated transcription",
  "term_id": "GO:0045892",
  "gene_symbol": "ZNF639",
  "gene": "UniProtKB:Q9UID6",
  "gene_name": "Zinc finger protein 639"
}